{
  "gene_symbol": "NXPH4",
  "term_id": "GO:0005102",
  "term_label": "signaling receptor binding",
  "gene_name": "Neurexophilin-4",
  "gene": "UniProtKB:O95158"
}